{
  "gene_name": "Chromodomain-helicase-DNA-binding protein 4",
  "term_id": "GO:0006338",
  "gene_symbol": "CHD4",
  "gene": "UniProtKB:Q14839",
  "term_label": "chromatin remodeling"
}